{
  "gene": "UniProtKB:Q9P121",
  "term_label": "heterophilic cell-cell adhesion",
  "term_id": "GO:0007157",
  "gene_symbol": "NTM",
  "gene_name": "Neurotrimin"
}